polar tube [GO:0044099] (cellular component) Relationships: is a type of cellular anatomical structure [GO:0110165] References: PMID:12076771, PMID:9723921 Sources: GOC:mf Definition: A highly specialized structure unique to microsporidia that is required for host cell invasion. In the spore, the polar tube is connected at the anterior end, and then coils around the sporoplasm. Upon appropriate environmental stimulation, the polar tube rapidly discharges out of the spore, pierces a cell membrane and serves as a conduit for sporoplasm passage into the new host cell.